{
  "term_label": "mitochondrial L-ornithine transmembrane transport",
  "gene_name": "Mitochondrial basic amino acids transporter",
  "gene_symbol": "SLC25A29",
  "term_id": "GO:1990575",
  "gene": "UniProtKB:Q8N8R3"
}